inositol metabolic process [GO:0006020] (biological process) Subtypes: inositol biosynthetic process [GO:0006021], inositol catabolic process [GO:0019310] Sources: ISBN:0198547684 Also known as: inositol metabolism, vitamin Bh metabolic process, vitamin Bh metabolism, myo-inositol metabolic process, myo-inositol metabolism Relationships: is a type of polyol metabolic process [GO:0019751] Definition: The chemical reactions and pathways involving inositol, 1,2,3,4,5,6-cyclohexanehexol, a growth factor for animals and microorganisms.